{
  "term_label": "Golgi apparatus",
  "gene": "UniProtKB:Q12893",
  "gene_name": "Transmembrane protein 115",
  "term_id": "GO:0005794",
  "gene_symbol": "TMEM115"
}